{
  "term_label": "regulation of transcription by RNA polymerase II",
  "gene": "UniProtKB:P41970",
  "gene_name": "ETS domain-containing protein Elk-3",
  "term_id": "GO:0006357",
  "gene_symbol": "ELK3"
}